{
  "gene_name": "Wilms tumor protein 1-interacting protein",
  "term_label": "regulation of DNA-templated transcription",
  "term_id": "GO:0006355",
  "gene": "UniProtKB:A6NIX2",
  "gene_symbol": "WTIP"
}